{
  "gene_name": "Glycylpeptide N-tetradecanoyltransferase 1",
  "gene": "UniProtKB:P30419",
  "term_label": "glycylpeptide N-tetradecanoyltransferase activity",
  "term_id": "GO:0004379",
  "gene_symbol": "NMT1"
}